post-translational protein modification [GO:0043687] (biological process) Also known as: PTM, post-translational amino acid modification, post-translational modification, posttranslational amino acid modification, posttranslational modification, posttranslational protein modification Relationships: is a type of protein modification process [GO:0036211] Regulation: RO_0002211 by regulation of post-translational protein modification [GO:1901873]; negatively regulated by negative regulation of post-translational protein modification [GO:1901874]; positively regulated by GO:1901875 Note: This term should only be used to annotate a protein modification process that occurs after the protein has been released from the ribosome, and is therefore strictly post-translational. Modification of a free protein (one not attached to a ribosome) and modification of a C-terminal residue are post-translational processes. Some protein modifications occur while the protein is still in the ribosome but before translation has been completed; these modification processes are considered co-translational and should not be annotated using this term. Definition: The process of covalently altering one or more amino acids in a protein after the protein has been completely translated and released from the ribosome. Sources: GOC:jsg Subtypes: C-terminal protein amino acid modification [GO:0018410], GO:0034421, N-terminal protein amino acid propionylation [GO:0061606], GO:0070212, protein auto-ADP-ribosylation [GO:0070213], GO:0070647